{
  "term_id": "GO:0017056",
  "gene": "UniProtKB:O75694",
  "term_label": "structural constituent of nuclear pore",
  "gene_name": "Nuclear pore complex protein Nup155",
  "gene_symbol": "NUP155"
}